{
  "term_label": "mitochondrial fission",
  "term_id": "GO:0000266",
  "gene": "UniProtKB:O00429",
  "gene_name": "Dynamin-1-like protein",
  "gene_symbol": "DNM1L"
}